{
  "term_label": "hormone-mediated signaling pathway",
  "gene_symbol": "RXFP1",
  "term_id": "GO:0009755",
  "gene_name": "Relaxin receptor 1",
  "gene": "UniProtKB:Q9HBX9"
}